{
  "term_label": "ubiquitin-protein transferase activity",
  "term_id": "GO:0004842",
  "gene": "UniProtKB:Q9UMS4",
  "gene_name": "Pre-mRNA-processing factor 19",
  "gene_symbol": "PRPF19"
}